{
  "term_label": "Unknown cellular component",
  "gene_symbol": "OR11H2",
  "gene_name": "Olfactory receptor 11H2",
  "gene": "UniProtKB:Q8NH07",
  "term_id": "UNKNOWN:0003"
}